{
  "term_label": "translation",
  "term_id": "GO:0006412",
  "gene": "UniProtKB:P15170",
  "gene_name": "Eukaryotic peptide chain release factor GTP-binding subunit ERF3A",
  "gene_symbol": "GSPT1"
}